{
  "term_label": "Unknown biological process",
  "gene_name": "Myosin light chain 5",
  "gene": "UniProtKB:Q02045",
  "gene_symbol": "MYL5",
  "term_id": "UNKNOWN:0002"
}